{
  "term_id": "GO:0005886",
  "term_label": "plasma membrane",
  "gene_name": "NT-3 growth factor receptor",
  "gene_symbol": "NTRK3",
  "gene": "UniProtKB:Q16288"
}